NarGHI complex [GO:0044799] (cellular component) Definition: A heterotrimeric protein complex with iron-sulfur and molybdenum cofactors that functions as a terminal reductase in electron transport pathways that operate during anaerobic nitrate respiration. In E. coli electrons are passed from the FdnGHI complex to the NarGHI complex via menoquinone and menaquinol. Within NarGHI, electrons are passed from the two heme molecules in the NarI subunit down a Fe-S cluster chain in the NarH and NarG subunits to the Molybdenum cofactor, Mo-bisMGD, in the NarG subunit. Also known as: cytoplasmic membrane-bound quinol-nitrate oxidoreductase, nitrate reductase A References: PMID:11289299, PMID:12910261, PMID:17964535 Sources: GOC:bhm Relationships: is_a nitrate reductase complex [GO:0009325]; is a type of GO:0098797; is a type of respiratory chain complex [GO:0098803]